B cell antigen processing and presentation mediated by B cell receptor uptake of antigen [GO:0002417] (biological process) Also known as: B lymphocyte antigen processing and presentation mediated by B cell receptor uptake of antigen, B-cell antigen processing and presentation mediated by B cell receptor uptake of antigen, B-lymphocyte antigen processing and presentation mediated by B cell receptor uptake of antigen Relationships: is a type of B cell antigen processing and presentation [GO:0002450]; is a type of GO:0002751 Definition: B cell antigen processing and presentation which is initiated by uptake of antigen bound to the B cell receptor. References: PMID:15771591 Sources: GOC:add, ISBN:0781735149